{
  "term_id": "GO:0006357",
  "term_label": "regulation of transcription by RNA polymerase II",
  "gene_symbol": "FOSL2",
  "gene_name": "Fos-related antigen 2",
  "gene": "UniProtKB:P15408"
}